{
  "gene": "UniProtKB:P0CG29",
  "gene_symbol": "GSTT2",
  "term_id": "GO:0004364",
  "term_label": "glutathione transferase activity",
  "gene_name": "Glutathione S-transferase theta-2"
}